{
  "gene_symbol": "CORT",
  "term_label": "G protein-coupled receptor binding",
  "gene": "UniProtKB:O00230",
  "gene_name": "Cortistatin",
  "term_id": "GO:0001664"
}